{
  "gene_name": "Protein FAM25C",
  "gene_symbol": "FAM25C",
  "term_label": "Unknown molecular function",
  "gene": "UniProtKB:B3EWG5",
  "term_id": "UNKNOWN:0001"
}